{
  "gene_symbol": "KISS1R",
  "gene": "UniProtKB:Q969F8",
  "term_label": "plasma membrane",
  "gene_name": "KiSS-1 receptor",
  "term_id": "GO:0005886"
}